{
  "gene_symbol": "RPL29",
  "gene_name": "Large ribosomal subunit protein eL29",
  "term_id": "GO:0022625",
  "gene": "UniProtKB:P47914",
  "term_label": "cytosolic large ribosomal subunit"
}